regulation of heart rate by chemical signal [GO:0003062] (biological process) Also known as: chemical cardiac chronotropy, chemical signal regulation of heart rate, chemical signal regulation of heart contraction rate Subtypes: negative regulation of heart rate by acetylcholine [GO:0003063], regulation of heart rate by hormone [GO:0003064], GO:0003065, positive regulation of heart rate by norepinephrine [GO:0003066] Definition: The regulation of the rate of heart contraction mediated by chemical signaling, hormonal, autocrine or paracrine. Relationships: is a type of GO:0002027 Sources: GOC:dph, GOC:mtg_cardio, GOC:rl, GOC:tb